epicardium-derived cardiac vascular smooth muscle cell fate commitment [GO:0060985] (biological process) Relationships: is a type of cardiac vascular smooth muscle cell fate commitment [GO:0060949]; is part of epicardium-derived cardiac vascular smooth muscle cell differentiation [GO:0060983] Sources: GOC:mtg_heart Definition: The commitment of an epicardial cell to a cardiac vascular smooth muscle cell fate and its capacity to differentiate into a cardiac vascular smooth muscle cell.